catechol O-methyltransferase activity [GO:0016206] (molecular function) Also known as: COMT I, COMT II, MB-COMT (membrane-bound form of catechol-O-methyltransferase), S-COMT (soluble form of catechol-O-methyltransferase), S-adenosyl-L-methionine:catechol O-methyltransferase activity, catechol methyltransferase activity, catecholamine O-methyltransferase activity Sources: EC:2.1.1.6, RHEA:17877 Definition: Catalysis of the reaction: a catechol + S-adenosyl-L-methionine = a guaiacol + H+ + S-adenosyl-L-homocysteine. Acts on catechols and on catecholamines such as adrenaline or noradrenaline. Relationships: is a type of O-methyltransferase activity [GO:0008171]; is a type of GO:0008757